{
  "gene_symbol": "QTRT2",
  "gene_name": "Queuine tRNA-ribosyltransferase accessory subunit 2",
  "gene": "UniProtKB:Q9H974",
  "term_id": "UNKNOWN:0003",
  "term_label": "Unknown cellular component"
}